{
  "gene_name": "DNA repair-scaffolding protein",
  "gene": "UniProtKB:Q14159",
  "term_label": "nucleoplasm",
  "term_id": "GO:0005654",
  "gene_symbol": "SPIDR"
}